{
  "term_id": "UNKNOWN:0002",
  "gene_name": "Muskelin",
  "gene": "UniProtKB:Q9UL63",
  "term_label": "Unknown biological process",
  "gene_symbol": "MKLN1"
}